{
  "gene": "UniProtKB:Q8N6W0",
  "gene_symbol": "CELF5",
  "gene_name": "CUGBP Elav-like family member 5",
  "term_label": "cytoplasm",
  "term_id": "GO:0005737"
}